{
  "gene_name": "Beta-1,3-glucosyltransferase",
  "term_id": "GO:0008375",
  "gene": "UniProtKB:Q6Y288",
  "term_label": "acetylglucosaminyltransferase activity",
  "gene_symbol": "B3GLCT"
}